{
  "term_id": "GO:0006955",
  "gene_symbol": "IGLV6-57",
  "gene_name": "Immunoglobulin lambda variable 6-57",
  "term_label": "immune response",
  "gene": "UniProtKB:P01721"
}